{
  "term_label": "Unknown biological process",
  "gene_name": "Thyroid peroxidase",
  "gene": "UniProtKB:P07202",
  "gene_symbol": "TPO",
  "term_id": "UNKNOWN:0002"
}